{
  "term_id": "GO:0061630",
  "term_label": "ubiquitin protein ligase activity",
  "gene_name": "Probable E3 ubiquitin-protein ligase DTX3",
  "gene": "UniProtKB:Q8N9I9",
  "gene_symbol": "DTX3"
}